{
  "term_id": "GO:0031146",
  "term_label": "SCF-dependent proteasomal ubiquitin-dependent protein catabolic process",
  "gene": "UniProtKB:Q5FWF7",
  "gene_name": "F-box only protein 48",
  "gene_symbol": "FBXO48"
}